{
  "gene": "UniProtKB:Q9Y2Y9",
  "gene_name": "Krueppel-like factor 13",
  "term_id": "GO:0000978",
  "gene_symbol": "KLF13",
  "term_label": "RNA polymerase II cis-regulatory region sequence-specific DNA binding"
}